{
  "gene_name": "IQ domain-containing protein F3",
  "gene": "UniProtKB:P0C7M6",
  "gene_symbol": "IQCF3",
  "term_id": "GO:0005516",
  "term_label": "calmodulin binding"
}